response to formic acid [GO:1901425] (biological process) Relationships: is a type of GO:1901700 Regulation: regulated by regulation of response to formic acid [GO:1901460]; negatively regulated by GO:1901461; positively regulated by positive regulation of response to formic acid [GO:1901462] Sources: GOC:TermGenie, GOC:mengo_curators Definition: Any process that results in a change in state or activity of a cell or an organism (in terms of movement, secretion, enzyme production, gene expression, etc.) as a result of a formic acid stimulus.